regulation of macrophage fusion [GO:0034239] (biological process) Subtypes: GO:0034240, GO:0034241 Relationships: is a type of regulation of syncytium formation by plasma membrane fusion [GO:0060142]; regulates macrophage fusion [GO:0034238] Definition: Any process that modulates the frequency, rate or extent of macrophage fusion. Sources: GOC:mah